teichoic acid biosynthetic process [GO:0019350] (biological process) Relationships: is a type of GO:0016053; is a type of cell wall macromolecule biosynthetic process [GO:0044038]; is a type of teichoic acid metabolic process [GO:0046374]; is a type of carbohydrate derivative biosynthetic process [GO:1901137]; BFO_0000050 GO:0009273 Also known as: teichoic acid anabolism, teichoic acid biosynthesis, teichoic acid formation, teichoic acid synthesis Sources: ISBN:0198506732 Definition: The chemical reactions and pathways resulting in the formation of teichoic acid, any polymer occurring in the cell wall, membrane or capsule of Gram-positive bacteria and containing chains of glycerol phosphate or ribitol phosphate residues. Subtypes: lipoteichoic acid biosynthetic process [GO:0070395], wall teichoic acid biosynthetic process [GO:0070398], teichoic acid D-alanylation [GO:0070400], poly(ribitol phosphate) teichoic acid biosynthetic process [GO:1902012], GO:1902014, poly(glucopyranosyl N-acetylgalactosamine 1-phosphate) teichoic acid biosynthetic process [GO:1902016]